{
  "term_label": "nucleoplasm",
  "gene": "UniProtKB:P62993",
  "gene_name": "Growth factor receptor-bound protein 2",
  "gene_symbol": "GRB2",
  "term_id": "GO:0005654"
}